{
  "term_id": "UNKNOWN:0001",
  "gene_name": "Small integral membrane protein 22",
  "term_label": "Unknown molecular function",
  "gene": "UniProtKB:K7EJ46",
  "gene_symbol": "SMIM22"
}